{
  "gene_name": "Pentraxin-related protein PTX3",
  "term_id": "GO:0001849",
  "term_label": "complement component C1q complex binding",
  "gene": "UniProtKB:P26022",
  "gene_symbol": "PTX3"
}